{
  "term_id": "GO:0004181",
  "gene_symbol": "CPA2",
  "term_label": "metallocarboxypeptidase activity",
  "gene": "UniProtKB:P48052",
  "gene_name": "Carboxypeptidase A2"
}